extrinsic component of endosome membrane [GO:0031313] (cellular component) Sources: GOC:dos, GOC:mah Subtypes: extrinsic component of postsynaptic endosome membrane [GO:0098999], extrinsic component of presynaptic endosome membrane [GO:0099007] Also known as: extrinsic to endosome membrane Relationships: is a type of extrinsic component of organelle membrane [GO:0031312]; is part of endosome membrane [GO:0010008] Definition: The component of an endosome membrane consisting of gene products and protein complexes that are loosely bound to one of its surfaces, but not integrated into the hydrophobic region.